{
  "gene": "UniProtKB:Q9P225",
  "term_id": "GO:0045505",
  "gene_symbol": "DNAH2",
  "gene_name": "Dynein axonemal heavy chain 2",
  "term_label": "dynein intermediate chain binding"
}